positive regulation of carbohydrate metabolic process [GO:0045913] (biological process) Also known as: positive regulation of carbohydrate metabolism, up regulation of carbohydrate metabolic process, up-regulation of carbohydrate metabolic process, upregulation of carbohydrate metabolic process, activation of carbohydrate metabolic process, stimulation of carbohydrate metabolic process Sources: GOC:go_curators Relationships: is a type of GO:0006109; is a type of positive regulation of metabolic process [GO:0009893]; positively regulates carbohydrate metabolic process [GO:0005975] Definition: Any process that activates or increases the frequency, rate or extent of the chemical reactions and pathways involving carbohydrate. Subtypes: positive regulation of glucose metabolic process [GO:0010907], positive regulation of glycolytic process [GO:0045821], positive regulation of (1->3)-beta-D-glucan biosynthetic process [GO:0060635], positive regulation of inositol phosphate biosynthetic process [GO:0060732], positive regulation of capsule polysaccharide biosynthetic process [GO:0062085], positive regulation of raffinose biosynthetic process [GO:1900093], positive regulation of hyaluronan biosynthetic process [GO:1900127], positive regulation of cellobiose catabolic process [GO:1900284], positive regulation of xylose catabolic process to ethanol [GO:1900517], positive regulation of trehalose catabolic process [GO:1901319], positive regulation of lactose biosynthetic process [GO:1903536], positive regulation of glyoxylate cycle [GO:2000876], positive regulation of starch catabolic process [GO:2000883], GO:2000914, positive regulation of cellodextrin catabolic process [GO:2000929], positive regulation of cellotriose catabolic process [GO:2000938], GO:2000959, positive regulation of cellooligosaccharide catabolic process [GO:2000965], positive regulation of cell wall polysaccharide catabolic process [GO:2000968], GO:2000990, positive regulation of galactomannan catabolic process [GO:2000993], positive regulation of cellulose catabolic process [GO:2000999], positive regulation of pectin catabolic process [GO:2001005], GO:2001008